nucleotide-excision repair, preincision complex [GO:0097520] (cellular component) Definition: A multiprotein complex involved in damage recognition, DNA helix unwinding, and endonucleolytic cleavage at the site of DNA damage. References: PMID:10197977 Sources: GOC:cjm, GOC:elh Also known as: UvrA(2)-UvrB(2) complex, UvrA(2)B(2) complex, UvrB dimer Relationships: is a type of protein-DNA complex [GO:0032993]